{
  "gene": "UniProtKB:Q96BM0",
  "gene_symbol": "IFI27L1",
  "term_label": "intrinsic apoptotic signaling pathway",
  "gene_name": "Interferon alpha-inducible protein 27-like protein 1",
  "term_id": "GO:0097193"
}